{
  "term_label": "regulation of transcription by RNA polymerase II",
  "gene": "UniProtKB:Q13422",
  "gene_name": "DNA-binding protein Ikaros",
  "term_id": "GO:0006357",
  "gene_symbol": "IKZF1"
}